{
  "gene_name": "Aryl hydrocarbon receptor nuclear translocator",
  "gene_symbol": "ARNT",
  "gene": "UniProtKB:P27540",
  "term_id": "GO:0005634",
  "term_label": "nucleus"
}